positive regulation of mitochondrial mRNA catabolic process [GO:1905639] (biological process) Relationships: is a type of positive regulation of mitochondrial RNA catabolic process [GO:0000962]; is a type of positive regulation of mRNA catabolic process [GO:0061014]; is_a regulation of mitochondrial mRNA catabolic process [GO:1905637]; positively regulates mitochondrial mRNA catabolic process [GO:0000958] Also known as: up regulation of mitochondrial mRNA catabolic process, up-regulation of mitochondrial mRNA catabolic process, upregulation of mitochondrial mRNA catabolic process, activation of mitochondrial mRNA catabolic process References: PMID:27122350 Sources: GOC:TermGenie, GO_REF:0000058 Definition: Any process that activates or increases the frequency, rate or extent of mitochondrial mRNA catabolic process.